mesonephric glomerular mesangial cell proliferation involved in mesonephros development [GO:0061269] (biological process) Regulation: regulated by regulation of mesonephric glomerular mesangial cell proliferation [GO:2000090]; RO_0002212 by negative regulation of mesonephric glomerular mesangial cell proliferation [GO:2000091]; positively regulated by positive regulation of mesonephric glomerular mesangial cell proliferation [GO:2000092] Sources: GOC:mtg_kidney_jan10 Relationships: is a type of cell proliferation involved in mesonephros development [GO:0061209]; is a type of GO:0072110; is part of mesonephric glomerular mesangium development [GO:0061247] Subtypes: mesonephric intraglomerular mesangial cell proliferation [GO:0061270] Definition: The multiplication or reproduction of glomerular mesangial cells in the mesonephros, resulting in the expansion of the population.